actin filament debranching activity [GO:0140775] (molecular function) Definition: Binding to an actin filament and promoting the dissociation of an actin filament branch. Also known as: actin debranching activity Relationships: is_a protein-containing complex destabilizing activity [GO:0140776]; BFO_0000050 actin cytoskeleton organization [GO:0030036]; has part actin filament binding [GO:0051015] References: PMID:20362448